symbiont-mediated suppression of host cytoplasmic pattern recognition receptor signaling pathway via inhibition of RIG-I activity [GO:0039540] (biological process) References: PMID:19454348, PMID:26138103 Note: This term is for annotation of symbiont proteins that counteract the host anti-microbial innate immune response initiated by host RIG-I, either by binding and inhibiting host RIG-I directly, or by interfering with other processes so that RIG-I is unable to carry out its normal function (e.g. by processing viral RNA so it cannot be recognized by RIG-I, or by promoting the degradation of RIG-I). Definition: A process in which a symbiont interferes with, inhibits or disrupts a cytoplasmic pattern recognition receptor signaling pathway by inhibiting the activity of RIG-1 (also known as DDX58). The cytoplasmic pattern recognition RIG-I recognizes viral RNA synthesized during active viral replication and signals to protect the host against viral infection, for example by inducing the expression of antiviral cytokines. Relationships: is_a symbiont-mediated suppression of cytoplasmic pattern recognition receptor signaling pathway [GO:0039537] Also known as: inhibition of host DDX58/RIG-I by virus, suppression by virus of host RIG-I signalling pathway, suppression by virus of host viral-induced cytoplasmic pattern recognition receptor signaling pathway via inhibition of host RIG-I activity, inhibition by virus of host DDX58 activity, inhibition by virus of host RIG-I, inhibition by virus of host RIG-I signaling, suppression by virus of host DDX58 signaling pathway, suppression by virus of host RIG-I activity, suppression by virus of host RIG-I signaling pathway, symbiont-mediated suppression of host RIG-I signaling pathway